{
  "gene_name": "BAG family molecular chaperone regulator 4",
  "gene_symbol": "BAG4",
  "term_id": "GO:0016020",
  "term_label": "membrane",
  "gene": "UniProtKB:O95429"
}